fermentation [GO:0006113] (BP) Regulation: regulated by regulation of fermentation [GO:0043465]; negatively regulated by negative regulation of fermentation [GO:1901003] Relationships: is_a energy derivation by oxidation of organic compounds [GO:0015980] Definition: The metabolic process that uses oxidation-reduction reactions of organic compounds and substrate-level phosphorylation for the generation of adenosine triphosphate (ATP), without consuming oxygen and is independent of electron transport chains. Subtypes: GO:0019653, glucose catabolic process to lactate [GO:0019659], GO:0019662, GO:0019665, GO:0030645, malolactic fermentation [GO:0043464], GO:0043466, D-xylose catabolic process to ethanol [GO:0044577], fermentative hydrogen production [GO:0044812], GO:1901089 References: PMID:25617754, PMID:38821505 Note: PMID:38821505 mentions exceptions regarding organic compounds and ETC. Fermentation sub-processes exclude glycolysis to prevent redundancy with the glycolytic pathway.